protein palmitoylation [GO:0018345] (biological process) Relationships: is a type of GO:0006497; is a type of protein acylation [GO:0043543] Subtypes: N-terminal protein palmitoylation [GO:0006500], peptidyl-L-cysteine S-palmitoylation [GO:0018230] References: PMID:15520806 Sources: GOC:jl Also known as: protein amino acid palmitoylation Definition: The covalent attachment of a palmitoyl group to a protein.